lactone catabolic process [GO:1901335] (biological process) Definition: The chemical reactions and pathways resulting in the breakdown of lactone. Relationships: is a type of catabolic process [GO:0009056]; is a type of lactone metabolic process [GO:1901334] Also known as: lactone breakdown, lactone catabolism, lactone degradation Sources: GOC:TermGenie Subtypes: L-ascorbic acid catabolic process [GO:0019854], enterobactin catabolic process [GO:0046214], GO:1900556, GO:1900801, erythromycin catabolic process [GO:1901114], GO:1901511, pentalenolactone catabolic process [GO:1901779]